{
  "gene_symbol": "PMEPA1",
  "gene": "UniProtKB:Q969W9",
  "gene_name": "Protein TMEPAI",
  "term_label": "early endosome membrane",
  "term_id": "GO:0031901"
}